{
  "term_label": "synapse",
  "term_id": "GO:0045202",
  "gene": "UniProtKB:Q96A49",
  "gene_name": "Synapse-associated protein 1",
  "gene_symbol": "SYAP1"
}